{
  "gene_name": "T cell receptor alpha joining 56 (Fragment)",
  "term_id": "UNKNOWN:0001",
  "gene_symbol": "TRAJ56",
  "term_label": "Unknown molecular function",
  "gene": "UniProtKB:A0A075B6Z2"
}